protein localization to uropod [GO:0036052] (BP) Definition: A process in which a protein is transported to, or maintained in, a uropod. A uropod is a membrane projection with related cytoskeletal components at the trailing edge of a migrating cell. Relationships: is_a protein localization to trailing edge [GO:0036051] References: PMID:12714569, PMID:12787750 Sources: GOC:add, GOC:pf, ISBN:0781735149 Also known as: protein localisation to uropod